{
  "term_id": "GO:0150105",
  "term_label": "protein localization to cell-cell junction",
  "gene_name": "Tight junction protein ZO-2",
  "gene": "UniProtKB:Q9UDY2",
  "gene_symbol": "TJP2"
}